microglia differentiation [GO:0014004] (biological process) Definition: The process in which a relatively unspecialized cell acquires specialized features of a microglial cell. Microglia are glial cells that act as the immune cells of the central nervous system. They form part of the supporting structure of this system. Sources: GOC:ef Also known as: microglial cell differentiation Relationships: is a type of glial cell differentiation [GO:0010001]; is a type of macrophage differentiation [GO:0030225]; is part of GO:0007417 Regulation: regulated by GO:0014006; negatively regulated by negative regulation of microglia differentiation [GO:0014007]; positively regulated by GO:0014008